{
  "term_label": "translation repressor activity",
  "gene_name": "Polyadenylate-binding protein-interacting protein 2",
  "gene_symbol": "PAIP2",
  "gene": "UniProtKB:Q9BPZ3",
  "term_id": "GO:0030371"
}